{
  "term_label": "structural constituent of ribosome",
  "term_id": "GO:0003735",
  "gene_symbol": "MRPL57",
  "gene_name": "Large ribosomal subunit protein mL63",
  "gene": "UniProtKB:Q9BQC6"
}